diphosphoinositol-polyphosphate diphosphatase activity [GO:0008486] (molecular function) Also known as: diphospho-myo-inositol-polyphosphate diphosphohydrolase activity, diphosphoinositol polyphosphate phosphohydrolase activity, diphosphoinositol-polyphosphate phosphohydrolase activity, DIPP activity Relationships: is a type of pyrophosphatase activity [GO:0016462] Sources: EC:3.6.1.52 Subtypes: GO:0052840, inositol bisdiphosphate tetrakisphosphate diphosphatase activity [GO:0052841], GO:0052842 Definition: Catalysis of the reaction: diphospho-1D-myo-inositol polyphosphate + H2O = 1D-myo-inositol polyphosphate + phosphate.